negative regulation of purine nucleotide catabolic process [GO:0033122] (biological process) Definition: Any process that stops, prevents, or reduces the frequency, rate or extent of the chemical reactions and pathways resulting in the breakdown of purine nucleotides. Subtypes: negative regulation of glycolytic process [GO:0045820] Also known as: negative regulation of purine nucleotide breakdown, negative regulation of purine nucleotide catabolism, negative regulation of purine nucleotide degradation Relationships: is a type of GO:0030812; is a type of GO:0033121; is a type of negative regulation of purine nucleotide metabolic process [GO:1900543]; negatively regulates purine nucleotide catabolic process [GO:0006195] Sources: GOC:mah